{
  "gene_name": "RalBP1-associated Eps domain-containing protein 2",
  "gene_symbol": "REPS2",
  "gene": "UniProtKB:Q8NFH8",
  "term_label": "protein-macromolecule adaptor activity",
  "term_id": "GO:0030674"
}